sensory organ boundary specification [GO:0008052] (BP) Also known as: sense organ boundary specification Definition: The process in which boundaries between a sensory organ and the surrounding tissue are established and maintained. Sources: GO_REF:0000021 Relationships: is a type of formation of animal organ boundary [GO:0010160]; is part of GO:0007423